{
  "gene_symbol": "OTX1",
  "gene": "UniProtKB:P32242",
  "term_label": "regulation of transcription by RNA polymerase II",
  "gene_name": "Homeobox protein OTX1",
  "term_id": "GO:0006357"
}